{
  "gene_name": "Peripheral-type benzodiazepine receptor-associated protein 1",
  "term_id": "GO:0030156",
  "term_label": "benzodiazepine receptor binding",
  "gene_symbol": "TSPOAP1",
  "gene": "UniProtKB:O95153"
}